{
  "gene_symbol": "PXDNL",
  "gene_name": "Probable oxidoreductase PXDNL",
  "gene": "UniProtKB:A1KZ92",
  "term_id": "GO:0005615",
  "term_label": "extracellular space"
}